negative regulation of vesicle transport along microtubule [GO:1901609] (biological process) Definition: Any process that stops, prevents or reduces the frequency, rate or extent of vesicle transport along microtubule. Sources: GOC:TermGenie Relationships: is a type of negative regulation of intracellular transport [GO:0032387]; is a type of regulation of vesicle transport along microtubule [GO:1901608]; RO_0002212 vesicle transport along microtubule [GO:0047496] Also known as: down regulation of microtubule-based vesicle localization, down regulation of vesicle transport along microtubule, down-regulation of microtubule-based vesicle localization, down-regulation of vesicle transport along microtubule, downregulation of microtubule-based vesicle localization, downregulation of vesicle transport along microtubule, inhibition of microtubule-based vesicle localization, negative regulation of microtubule-based vesicle localization, inhibition of vesicle transport along microtubule Subtypes: negative regulation of anterograde dense core granule transport [GO:1901952], negative regulation of retrograde dense core granule transport [GO:1901955], negative regulation of anterograde synaptic vesicle transport [GO:1903743]